2-dehydro-3-deoxygluconokinase activity [GO:0008673] (MF) Definition: Catalysis of the reaction: 2-dehydro-3-deoxy-D-gluconate + ATP = 2-dehydro-3-deoxy-6-phospho-D-gluconate + ADP + 2 H+. Sources: EC:2.7.1.45, RHEA:14797 Also known as: 2-keto-3-deoxy-D-gluconic acid kinase activity, 2-keto-3-deoxygluconate kinase activity, 2-keto-3-deoxygluconokinase (phosphorylating), 2-keto-3-deoxygluconokinase activity, 3-deoxy-2-oxo-D-gluconate kinase activity, ATP:2-dehydro-3-deoxy-D-gluconate 6-phosphotransferase activity, KDG kinase activity, ketodeoxygluconokinase activity Relationships: is a type of phosphotransferase activity, alcohol group as acceptor [GO:0016773]; is a type of GO:0019200